{
  "gene": "UniProtKB:P22310",
  "gene_symbol": "UGT1A4",
  "gene_name": "UDP-glucuronosyltransferase 1A4",
  "term_label": "enzyme binding",
  "term_id": "GO:0019899"
}